{
  "term_id": "GO:0005737",
  "term_label": "cytoplasm",
  "gene": "UniProtKB:Q96S59",
  "gene_name": "Ran-binding protein 9",
  "gene_symbol": "RANBP9"
}